{
  "term_id": "GO:0000122",
  "term_label": "negative regulation of transcription by RNA polymerase II",
  "gene": "UniProtKB:O95503",
  "gene_name": "Chromobox protein homolog 6",
  "gene_symbol": "CBX6"
}